gonad morphogenesis [GO:0035262] (biological process) Relationships: is a type of GO:0003006; is a type of animal organ morphogenesis [GO:0009887]; is part of GO:0008406 Definition: The process in which the anatomical structures of the gonads are generated and organized. A gonad is an animal organ producing gametes, e.g. the testes or the ovary in mammals. Subtypes: female gonad morphogenesis [GO:0061040] Sources: ISBN:0198612001